{
  "gene": "UniProtKB:Q9UIA0",
  "term_id": "GO:0005886",
  "gene_symbol": "CYTH4",
  "term_label": "plasma membrane",
  "gene_name": "Cytohesin-4"
}